{
  "gene_name": "Secretoglobin family 1D member 2",
  "gene": "UniProtKB:O95969",
  "term_id": "UNKNOWN:0001",
  "term_label": "Unknown molecular function",
  "gene_symbol": "SCGB1D2"
}